{
  "term_id": "UNKNOWN:0001",
  "gene_name": "Transmembrane protein 229B",
  "term_label": "Unknown molecular function",
  "gene": "UniProtKB:Q8NBD8",
  "gene_symbol": "TMEM229B"
}